copper ion sensor activity [GO:0097077] (molecular function) References: PMID:19928961 Sources: GOC:rs Relationships: is a type of metal ion sensor activity [GO:0140784]; has part copper ion binding [GO:0005507] Definition: Binding to and responding, e.g. by conformational change, to changes in the cellular level of copper(I) (Cu+).